regulation of programmed cell death [GO:0043067] (biological process) Also known as: regulation of non-apoptotic programmed cell death Sources: GOC:jl Relationships: is a type of regulation of cellular process [GO:0050794]; regulates programmed cell death [GO:0012501] Subtypes: regulation of plant-type hypersensitive response [GO:0010363], GO:0042981, positive regulation of programmed cell death [GO:0043068], negative regulation of programmed cell death [GO:0043069], regulation of retinal cell programmed cell death [GO:0046668], GO:0062098, GO:0110075, regulation of hydrogen peroxide-mediated programmed cell death [GO:1901298], regulation of autophagic cell death [GO:1904092], regulation of cornification [GO:1905715] Definition: Any process that modulates the frequency, rate or extent of programmed cell death, cell death resulting from activation of endogenous cellular processes.